{
  "gene": "UniProtKB:P34903",
  "gene_name": "Gamma-aminobutyric acid receptor subunit alpha-3",
  "term_label": "gamma-aminobutyric acid signaling pathway",
  "term_id": "GO:0007214",
  "gene_symbol": "GABRA3"
}